{
  "gene_name": "Transgelin",
  "term_id": "UNKNOWN:0002",
  "gene": "UniProtKB:Q01995",
  "gene_symbol": "TAGLN",
  "term_label": "Unknown biological process"
}